{
  "term_id": "UNKNOWN:0002",
  "gene": "UniProtKB:Q8N2Q7",
  "gene_name": "Neuroligin-1",
  "term_label": "Unknown biological process",
  "gene_symbol": "NLGN1"
}